{
  "gene_name": "Phosphatidylinositol 4-phosphate 3-kinase C2 domain-containing subunit beta",
  "gene": "UniProtKB:O00750",
  "term_id": "GO:0016477",
  "term_label": "cell migration",
  "gene_symbol": "PIK3C2B"
}